cell surface [GO:0009986] (cellular component) Sources: GOC:jl, GOC:mtg_sensu, GOC:sm Note: Note that this term is intended to annotate gene products that are attached (integrated or loosely bound) to the plasma membrane or cell wall. Definition: The external part of the cell wall and/or plasma membrane. Relationships: is a type of GO:0110165 Also known as: cell associated, cell bound